{
  "term_label": "chromatin binding",
  "term_id": "GO:0003682",
  "gene_symbol": "TSPY2",
  "gene_name": "Testis-specific Y-encoded protein 2",
  "gene": "UniProtKB:A6NKD2"
}